{
  "gene_symbol": "PHYHIPL",
  "term_id": "UNKNOWN:0002",
  "gene": "UniProtKB:Q96FC7",
  "term_label": "Unknown biological process",
  "gene_name": "Phytanoyl-CoA hydroxylase-interacting protein-like"
}